{
  "gene": "UniProtKB:Q9BY66",
  "term_id": "GO:0006338",
  "gene_symbol": "KDM5D",
  "term_label": "chromatin remodeling",
  "gene_name": "Lysine-specific demethylase 5D"
}